{
  "gene_name": "Putative protein SSX8",
  "term_id": "UNKNOWN:0001",
  "gene": "UniProtKB:Q7RTT4",
  "gene_symbol": "SSX8P",
  "term_label": "Unknown molecular function"
}